leukocyte adhesion to arterial endothelial cell [GO:0061757] (biological process) Relationships: is a type of GO:0061756 Definition: The attachment of a leukocyte to an arterial endothelial cell via adhesion molecules. Regulation: regulated by regulation of leukocyte adhesion to arterial endothelial cell [GO:1904997]; negatively regulated by GO:1904998; positively regulated by positive regulation of leukocyte adhesion to arterial endothelial cell [GO:1904999] References: PMID:22267480 Sources: GOC:BHF, GOC:BHF_miRNA, GOC:add, GOC:bc